{
  "term_id": "UNKNOWN:0003",
  "gene": "UniProtKB:Q9BQW3",
  "term_label": "Unknown cellular component",
  "gene_name": "Transcription factor COE4",
  "gene_symbol": "EBF4"
}